chorismate lyase activity [GO:0008813] (molecular function) Relationships: is a type of oxo-acid-lyase activity [GO:0016833] Definition: Catalysis of the reaction: chorismate = 4-hydroxybenzoate + pyruvate. Also known as: 4-hydroxybenzoate synthetase activity, chorismate pyruvate lyase activity, CL, CPL, UbiC, chorismate pyruvate-lyase (4-hydroxybenzoate-forming) activity Sources: EC:4.1.3.40, RHEA:16505